{
  "term_label": "serine-type endopeptidase inhibitor activity",
  "gene_name": "Angiotensinogen",
  "gene_symbol": "AGT",
  "term_id": "GO:0004867",
  "gene": "UniProtKB:P01019"
}